{
  "gene_symbol": "NEURL2",
  "gene_name": "Neuralized-like protein 2",
  "term_label": "ubiquitin protein ligase activity",
  "gene": "UniProtKB:Q9BR09",
  "term_id": "GO:0061630"
}